{
  "gene_name": "Dedicator of cytokinesis protein 11",
  "gene_symbol": "DOCK11",
  "term_label": "guanyl-nucleotide exchange factor activity",
  "gene": "UniProtKB:Q5JSL3",
  "term_id": "GO:0005085"
}